interleukin-15 receptor complex [GO:1905543] (cellular component) Definition: A protein complex that binds interleukin-15 (IL-15) and that consists of, at a minimum, an interleukin, an alpha, beta and gamma chain as well as optional additional kinase subunits. The alpha chain is unique to binds IL-15 while it shares the beta chain with the IL-2 receptor and the cytokine receptor common gamma chain with multiple interleukin receptors. References: PMID:23104097 Sources: GOC:TermGenie, GOC:bhm, GO_REF:0000088 Note: An example of this is IL15RA in human (Q13261) in PMID:23104097 (inferred from physical interaction). Relationships: is_a receptor complex [GO:0043235] Also known as: IL-15 receptor complex, IL-15-receptor complex, IL15 receptor complex, IL15-receptor complex, interleukin-15-receptor complex